protein-phosphocysteine-sugar phosphotransferase activity [GO:0090563] (molecular function) Relationships: is a type of carbohydrate transmembrane transporter activity [GO:0015144]; is a type of phosphotransferase activity, alcohol group as acceptor [GO:0016773]; is a type of active transmembrane transporter activity [GO:0022804] Sources: GOC:am Definition: Catalysis of the PEP-dependent, phosphoryl transfer-driven transport of substances across a membrane. The transport happens by catalysis of the reaction: protein S-phosphocysteine + sugar(out) = protein cysteine + sugar phosphate(in). This differs from primary and secondary active transport in that the solute is modified during transport. Subtypes: protein-phosphocysteine-glucose phosphotransferase system transporter activity [GO:0090564], GO:0090565, GO:0090566, GO:0090581, protein-phosphocysteine-D-fructose-phosphotransferase system transporter activity [GO:0090582], protein-phosphocysteine-D-sorbitol-phosphotransferase system transporter activity [GO:0090583], protein-phosphocysteine-galactitol-phosphotransferase system transporter activity [GO:0090584], GO:0090585, GO:0090586, protein-phosphocysteine-glucosamine phosphotransferase system transporter activity [GO:0090587], protein-phosphocysteine-N-acetylmuramate phosphotransferase system transporter activity [GO:0090588], protein-phosphocysteine-trehalose phosphotransferase system transporter activity [GO:0090589]